cleavage between SSU-rRNA and 5.8S rRNA of tetracistronic rRNA transcript (SSU-rRNA, 5.8S rRNA, 2S rRNA, LSU-rRNA) [GO:0000484] (biological process) Definition: Endonucleolytic cleavage between the SSU-rRNA and the 5.8S rRNA of an rRNA molecule originally produced as a tetracistronic rRNA transcript that contained the Small SubUnit (SSU) rRNA, the 5.8S rRNA, 2S rRNA, and the Large SubUnit (LSU) rRNA, in that order, from 5' to 3' along the primary transcript. Sources: GOC:curators Relationships: is a type of GO:0000483; is part of maturation of SSU-rRNA from tetracistronic rRNA transcript (SSU-rRNA, 5.8S rRNA, 2S rRNA, LSU-rRNA) [GO:0000474]; is part of GO:0000487